{
  "gene_symbol": "SUSD4",
  "term_id": "UNKNOWN:0001",
  "gene_name": "Sushi domain-containing protein 4",
  "gene": "UniProtKB:Q5VX71",
  "term_label": "Unknown molecular function"
}